{
  "term_label": "cytoplasmic vesicle",
  "gene_name": "DENN domain-containing protein 3",
  "term_id": "GO:0031410",
  "gene": "UniProtKB:A2RUS2",
  "gene_symbol": "DENND3"
}